structural constituent of albumen [GO:0097099] (MF) Definition: The action of a molecule that contributes to the structural integrity of albumen (also called egg white). Albumen is the clear liquid contained within an egg and consists of water and proteins, among which are ovomucin and ovomucoid. It protects the egg yolk and provides additional nutrition for the growth of the embryo. Also known as: structural constituent of egg white Relationships: is a type of structural molecule activity [GO:0005198] Sources: GOC:jj, Wikipedia:Albumen